{
  "gene_symbol": "USP8",
  "term_label": "Ras protein signal transduction",
  "gene": "UniProtKB:P40818",
  "term_id": "GO:0007265",
  "gene_name": "Ubiquitin carboxyl-terminal hydrolase 8"
}